{
  "gene_name": "Kinetochore scaffold 1",
  "gene_symbol": "KNL1",
  "gene": "UniProtKB:Q8NG31",
  "term_id": "GO:0008608",
  "term_label": "attachment of spindle microtubules to kinetochore"
}